MOZ/MORF histone acetyltransferase complex [GO:0070776] (cellular component) Definition: A histone acetyltransferase complex that has histone H3 acetyltransferase and coactivator activities. Subunits of the human complex include MYST3/MOZ, MYST4/MORF, ING5, EAF6 and one of BRPF1, BRD1/BRPF2 and BRPF3. Relationships: is a type of GO:0070775 References: PMID:18794358